{
  "gene": "UniProtKB:Q6UXN2",
  "gene_name": "Trem-like transcript 4 protein",
  "term_label": "positive regulation of toll-like receptor 7 signaling pathway",
  "gene_symbol": "TREML4",
  "term_id": "GO:0034157"
}